noradrenergic neuron fate commitment involved in brainstem development [GO:0003362] (biological process) Definition: The process in which the developmental fate of a cell becomes restricted such that it will develop into a noradrenergic neuron that is part of the brainstem. Sources: GOC:dph Relationships: is_a noradrenergic neuron fate commitment [GO:0003359]; is part of noradrenergic neuron differentiation involved in brainstem development [GO:0003361]